{
  "gene_name": "T-box transcription factor T",
  "gene_symbol": "TBXT",
  "gene": "UniProtKB:O15178",
  "term_label": "regulation of transcription by RNA polymerase II",
  "term_id": "GO:0006357"
}